negative regulation of heterochromatin organization [GO:0120262] (BP) Definition: Any process that stops, prevents, or reduces the frequency, rate or extent of heterochromatin organization. Also known as: down regulation of heterochromatin organization, down-regulation of heterochromatin organization, downregulation of heterochromatin organization, inhibition of heterochromatin organization Sources: GOC:krc Relationships: is a type of GO:0120261; is a type of negative regulation of chromatin organization [GO:1905268]; negatively regulates heterochromatin organization [GO:0070828]